{
  "term_label": "Unknown molecular function",
  "gene_name": "Protein ZNF767",
  "term_id": "UNKNOWN:0001",
  "gene": "UniProtKB:Q75MW2",
  "gene_symbol": "ZNF767P"
}